{
  "gene_name": "5'-AMP-activated protein kinase catalytic subunit alpha-2",
  "term_label": "protein localization to lipid droplet",
  "gene": "UniProtKB:P54646",
  "term_id": "GO:1990044",
  "gene_symbol": "PRKAA2"
}